{
  "gene_name": "Transcription factor SOX-6",
  "term_label": "nucleus",
  "term_id": "GO:0005634",
  "gene": "UniProtKB:P35712",
  "gene_symbol": "SOX6"
}